{
  "gene_symbol": "ABCG1",
  "term_id": "GO:0042632",
  "gene": "UniProtKB:P45844",
  "term_label": "cholesterol homeostasis",
  "gene_name": "ATP-binding cassette sub-family G member 1"
}